chromosomal 5-methylcytosine DNA demethylation, oxidative deamination pathway [GO:0141168] (biological process) References: PMID:21862972, PMID:29875631, PMID:36478523 Note: Note that this term describes one of the biochemical pathways of chromosomal cytosine demethylation but is agnostic to the effect on gene expression. If the data supports it, consider co-annotating to 'positive regulation of gene expression, epigenetic ; GO:0044029' or a child. A similar pathway may also convert chromosomal DNA N6-methyladenosine to adenosine but little evidence exists for this pathway. Current evidence indicates that this pathway in used for DNA repair, and not for epigenetic gene expression regulation. Also known as: epigenetic 5-methylcytosine DNA demethylation, oxidative deamination pathway, epigenetic DNA demethylation, oxidative deamination pathway Definition: An epigenetic cytosine DNA demethylation pathway that includes a deamination step to produce either a thymine (T), or a 5-hydroxymethyluracil (5hmU), if the 5meC had first been converted to 5hmC. A DNA glycosylase (e. g. TDG) recognizes the T mispaired with a G or the 5hmC and excises the modified base to initiate its replacement with unmethylated cytosine through base excision repair. Relationships: is a type of DNA repair [GO:0006281]; is a type of GO:0141166